{
  "term_id": "UNKNOWN:0001",
  "gene": "UniProtKB:Q14699",
  "term_label": "Unknown molecular function",
  "gene_symbol": "RFTN1",
  "gene_name": "Raftlin"
}